{
  "gene_name": "Integrator complex subunit 1",
  "gene_symbol": "INTS1",
  "gene": "UniProtKB:Q8N201",
  "term_id": "GO:0034474",
  "term_label": "U2 snRNA 3'-end processing"
}